{
  "gene_symbol": "FRG2C",
  "gene": "UniProtKB:A6NGY1",
  "term_label": "Unknown molecular function",
  "term_id": "UNKNOWN:0001",
  "gene_name": "Protein FRG2-like-2"
}